{
  "gene": "UniProtKB:Q9H7B4",
  "gene_symbol": "SMYD3",
  "term_label": "negative regulation of DNA-templated transcription",
  "term_id": "GO:0045892",
  "gene_name": "Histone-lysine N-methyltransferase SMYD3"
}